{
  "term_id": "UNKNOWN:0003",
  "gene_symbol": "MSANTD3",
  "gene_name": "Myb_SANT-like DNA-binding domain-containing protein 3",
  "term_label": "Unknown cellular component",
  "gene": "UniProtKB:Q96H12"
}